3-alpha-hydroxyglycyrrhetinate dehydrogenase activity [GO:0047032] (molecular function) Definition: Catalysis of the reaction: 3alpha-hydroxyglycyrrhetinate + NADP+ = 3-oxoglycyrrhetinate + H+ + NADPH. Sources: EC:1.1.1.230, RHEA:20816 Also known as: 3alpha-hydroxyglycyrrhetinate dehydrogenase activity, 3alpha-hydroxyglycyrrhetinate:NADP+ 3-oxidoreductase activity Relationships: is_a oxidoreductase activity, acting on the CH-OH group of donors, NAD or NADP as acceptor [GO:0016616]